{
  "gene_symbol": "HARBI1",
  "gene_name": "Putative nuclease HARBI1",
  "term_label": "Unknown biological process",
  "gene": "UniProtKB:Q96MB7",
  "term_id": "UNKNOWN:0002"
}